myoblast fate commitment [GO:0048625] (biological process) Sources: CL:0000056, GOC:dph, GOC:mtg_muscle Definition: The process in which the developmental fate of a cell becomes restricted such that it will develop into a myoblast. A myoblast is a mononucleate cell type that, by fusion with other myoblasts, gives rise to the myotubes that eventually develop into skeletal muscle fibers. Relationships: is a type of cell fate commitment [GO:0045165]; BFO_0000050 GO:0045445 Subtypes: myoblast fate commitment in head [GO:0014714], myoblast fate commitment in trunk [GO:0014715], myoblast fate commitment involved in skeletal muscle regeneration [GO:0014836]